adherens junction disassembly [GO:0120179] (biological process) Definition: The disaggregation of an adherens junction into its constituent components. An adherens junction is a cell-cell junction composed of the epithelial cadherin-catenin complex at which the cytoplasmic face of the plasma membrane is attached to actin filaments. Relationships: is_a adherens junction organization [GO:0034332]; is a type of cell-cell junction disassembly [GO:0150147] References: PMID:25490267 Sources: GOC:aruk, GOC:bc